{
  "term_label": "intracellular iron ion homeostasis",
  "gene": "UniProtKB:P49279",
  "term_id": "GO:0006879",
  "gene_symbol": "SLC11A1",
  "gene_name": "Natural resistance-associated macrophage protein 1"
}